{
  "gene": "UniProtKB:Q8TDF5",
  "term_label": "regulation of neurotransmitter receptor localization to postsynaptic specialization membrane",
  "term_id": "GO:0098696",
  "gene_symbol": "NETO1",
  "gene_name": "Neuropilin and tolloid-like protein 1"
}